{
  "gene_name": "Mitochondrial glutamate carrier 2",
  "gene_symbol": "SLC25A18",
  "term_label": "Unknown cellular component",
  "term_id": "UNKNOWN:0003",
  "gene": "UniProtKB:Q9H1K4"
}